{
  "term_id": "UNKNOWN:0002",
  "term_label": "Unknown biological process",
  "gene": "UniProtKB:A6NNL5",
  "gene_symbol": "C15orf61",
  "gene_name": "Uncharacterized protein C15orf61"
}